regulation of isotype switching to IgE isotypes [GO:0048293] (biological process) Definition: Any process that modulates the frequency, rate or extent of isotype switching to IgE isotypes. Sources: GOC:jid Also known as: regulation of class switch recombination to IgE isotypes, regulation of class switching to IgE isotypes, regulation of isotype switch recombination to IgE isotypes Relationships: is a type of GO:0045191; RO_0002211 GO:0048289 Subtypes: GO:0048294, positive regulation of isotype switching to IgE isotypes [GO:0048295], regulation of interleukin-4-dependent isotype switching to IgE isotypes [GO:2000571]